melibiose biosynthetic process [GO:0042544] (BP) Relationships: is a type of disaccharide biosynthetic process [GO:0046351] Definition: The chemical reactions and pathways resulting in the formation of melibiose, the disaccharide 6-O-alpha-D-galactopyranosyl-D-glucose. Sources: GOC:jl, ISBN:0198506732 Also known as: melibiose anabolism, melibiose biosynthesis, melibiose formation, melibiose synthesis